{
  "gene_name": "Dynein axonemal heavy chain 2",
  "gene_symbol": "DNAH2",
  "term_label": "dynein light intermediate chain binding",
  "term_id": "GO:0051959",
  "gene": "UniProtKB:Q9P225"
}